{
  "gene": "UniProtKB:P43366",
  "term_label": "negative regulation of transcription by RNA polymerase II",
  "gene_name": "Melanoma-associated antigen B1",
  "gene_symbol": "MAGEB1",
  "term_id": "GO:0000122"
}